{
  "gene": "UniProtKB:Q99538",
  "gene_name": "Legumain",
  "term_id": "GO:0051603",
  "term_label": "proteolysis involved in protein catabolic process",
  "gene_symbol": "LGMN"
}